{
  "gene_symbol": "CHRNA10",
  "term_label": "chemical synaptic transmission",
  "term_id": "GO:0007268",
  "gene_name": "Neuronal acetylcholine receptor subunit alpha-10",
  "gene": "UniProtKB:Q9GZZ6"
}